mitochondrial potassium ion transmembrane transport [GO:0140141] (biological process) Definition: The process in which a potassium ion is transported across a mitochondrial membrane, into or out of the mitochondrion. Relationships: is_a GO:0071805 References: PMID:20197279 Sources: GOC:vw